{
  "gene_name": "Acyl-CoA-binding domain-containing protein 6",
  "term_id": "UNKNOWN:0003",
  "term_label": "Unknown cellular component",
  "gene_symbol": "ACBD6",
  "gene": "UniProtKB:Q9BR61"
}